CDP-ribitol ribitolphosphotransferase activity [GO:0047356] (molecular function) Relationships: is a type of phosphotransferase activity, for other substituted phosphate groups [GO:0016780] Definition: Catalysis of the reaction: ribitol phosphate(n) + CDP-ribitol = ribitol phosphate(n+1) + CMP. Sources: EC:2.7.8.14 Also known as: teichoic-acid synthase activity, CDP-ribitol:poly(ribitol phosphate) ribitolphosphotransferase activity, CDPribitol ribitolphosphotransferase activity, poly(ribitol phosphate) synthetase activity, polyribitol phosphate polymerase activity, polyribitol phosphate synthetase activity, teichoate synthase activity, teichoate synthetase activity